{
  "term_id": "GO:0006457",
  "term_label": "protein folding",
  "gene": "UniProtKB:Q14318",
  "gene_name": "Peptidyl-prolyl cis-trans isomerase FKBP8",
  "gene_symbol": "FKBP8"
}